3'-N-debenzoyl-2'-deoxytaxol N-benzoyltransferase activity [GO:0102923] (molecular function) Relationships: is a type of acyltransferase activity, transferring groups other than amino-acyl groups [GO:0016747] Definition: Catalysis of the reaction: 3'-N-debenzoyltaxol + benzoyl-CoA = CoA + H+ + taxol. Sources: RHEA:33687